{
  "gene_name": "Chromobox protein homolog 6",
  "term_id": "GO:0035102",
  "gene_symbol": "CBX6",
  "term_label": "PRC1 complex",
  "gene": "UniProtKB:O95503"
}